{
  "gene_symbol": "DDX23",
  "gene_name": "Probable ATP-dependent RNA helicase DDX23",
  "term_label": "mRNA binding",
  "gene": "UniProtKB:Q9BUQ8",
  "term_id": "GO:0003729"
}